{
  "gene_symbol": "ZNF616",
  "gene": "UniProtKB:Q08AN1",
  "term_label": "nucleus",
  "term_id": "GO:0005634",
  "gene_name": "Zinc finger protein 616"
}